lateral ventricle development [GO:0021670] (biological process) Relationships: is a type of anatomical structure development [GO:0048856]; is part of telencephalon development [GO:0021537]; is part of ventricular system development [GO:0021591] Definition: The process whose specific outcome is the progression of the lateral ventricles over time, from the formation to the mature structure. The two lateral ventricles are a cavity in each of the cerebral hemispheres derived from the cavity of the embryonic neural tube. They are separated from each other by the septum pellucidum, and each communicates with the third ventricle by the foramen of Monro, through which also the choroid plexuses of the lateral ventricles become continuous with that of the third ventricle. Sources: GOC:cls, GOC:dgh, GOC:dph, GOC:jid, GO_REF:0000021